{
  "term_id": "UNKNOWN:0002",
  "gene_symbol": "DCAF4L1",
  "gene": "UniProtKB:Q3SXM0",
  "term_label": "Unknown biological process",
  "gene_name": "DDB1- and CUL4-associated factor 4-like protein 1"
}